nodal receptor complex [GO:0038104] (cellular component) Note: Nodal signals through activin receptors but (unlike activin) also requires EGF-CFC coreceptors (such as Cripto or Cryptic in mammals) to signal. This term is intended for receptor/co-receptor components and not a nodal-receptor complex. Also known as: ActRIIB.ALK4.EGF-CFC complex References: PMID:11024047, PMID:15062104 Sources: GOC:bf, GOC:signaling Definition: A protein complex containing at least a type II activin receptor, a type I activin receptor, and a coreceptor (EGF-CFC protein) such as Cripto or Cryptic. Nodal receptor complexes are capable of binding a nodal protein and transducing the signal into the cell. Relationships: is a type of receptor complex [GO:0043235]